{
  "term_id": "GO:1902358",
  "gene": "UniProtKB:Q9BZW2",
  "gene_symbol": "SLC13A1",
  "term_label": "sulfate transmembrane transport",
  "gene_name": "Solute carrier family 13 member 1"
}